heterotypic cell-cell adhesion [GO:0034113] (BP) Definition: The attachment of a cell to a cell of a different type via adhesion molecules. Sources: GOC:add Note: Note that this term is not synonymous with 'heterophilic cell adhesion ; GO:0007157'; the process may occur by homophilic or heterophilic mechanisms. Relationships: is a type of cell-cell adhesion [GO:0098609] Subtypes: GO:0086022, atrial cardiac muscle cell-AV node cell adhesion involved in cell communication [GO:0086071], GO:0086072, bundle of His cell-Purkinje myocyte adhesion involved in cell communication [GO:0086073], Purkinje myocyte-ventricular cardiac muscle cell adhesion involved in cell communication [GO:0086074], GO:0160015 Regulation: regulated by GO:0034114; negatively regulated by negative regulation of heterotypic cell-cell adhesion [GO:0034115]; positively regulated by positive regulation of heterotypic cell-cell adhesion [GO:0034116]